protein localization to motile cilium [GO:0120229] (biological process) Definition: A process in which a protein is transported to, or maintained in, a location within a motile cilium. Relationships: is a type of GO:0061512 Also known as: protein localization to nonmotile primary cilium References: PMID:27486780 Sources: GOC:krc